3-beta-hydroxy-5-alpha-steroid dehydrogenase (NADP+) activity [GO:0033704] (molecular function) Definition: Catalysis of the reaction: -3beta-hydroxy-5alpha-pregnane-20-one + NADP+ = 5-alpha-pregnane-3,20-dione + H+ + NADPH. Sources: RHEA:18137 Relationships: is a type of steroid dehydrogenase activity, acting on the CH-OH group of donors, NAD or NADP as acceptor [GO:0033764] Also known as: 3beta-hydroxy-5alpha-steroid:NADP+ 3-oxidoreductase activity